{
  "gene": "UniProtKB:P35712",
  "gene_name": "Transcription factor SOX-6",
  "term_id": "GO:0000981",
  "gene_symbol": "SOX6",
  "term_label": "DNA-binding transcription factor activity, RNA polymerase II-specific"
}